{
  "gene_name": "Probable phospholipid-transporting ATPase IIB",
  "gene_symbol": "ATP9B",
  "gene": "UniProtKB:O43861",
  "term_id": "GO:0005768",
  "term_label": "endosome"
}